{
  "gene_symbol": "SLC22A9",
  "gene": "UniProtKB:Q8IVM8",
  "term_label": "Unknown molecular function",
  "term_id": "UNKNOWN:0001",
  "gene_name": "Organic anion transporter 7"
}